{
  "gene_name": "Sulfotransferase 1C2",
  "term_id": "GO:0051923",
  "gene": "UniProtKB:O00338",
  "term_label": "sulfation",
  "gene_symbol": "SULT1C2"
}